{
  "gene": "UniProtKB:P55786",
  "term_label": "peptide catabolic process",
  "term_id": "GO:0043171",
  "gene_name": "Puromycin-sensitive aminopeptidase",
  "gene_symbol": "NPEPPS"
}